{
  "gene_name": "Plexin domain-containing protein 2",
  "gene": "UniProtKB:Q6UX71",
  "term_id": "UNKNOWN:0001",
  "gene_symbol": "PLXDC2",
  "term_label": "Unknown molecular function"
}